{
  "gene": "UniProtKB:Q8N7X1",
  "gene_name": "RNA-binding motif protein, X-linked-like-3",
  "term_label": "snRNA binding",
  "gene_symbol": "RBMXL3",
  "term_id": "GO:0017069"
}